{
  "gene": "UniProtKB:Q86W50",
  "gene_symbol": "METTL16",
  "term_label": "rRNA base methylation",
  "gene_name": "RNA N6-adenosine-methyltransferase METTL16",
  "term_id": "GO:0070475"
}